voltage-gated sodium channel activity involved in bundle of His cell action potential [GO:0086061] (molecular function) Definition: Enables the transmembrane transfer of a sodium ion by a voltage-gated channel through the plasma membrane of a bundle of His cardiac muscle cell contributing to the depolarization phase of an action potential. A voltage-gated channel is a channel whose open state is dependent on the voltage across the membrane in which it is embedded. Also known as: voltage-gated sodium channel activity involved in bundle of His cardiac muscle cell action potential Relationships: is a type of voltage-gated sodium channel activity involved in cardiac muscle cell action potential [GO:0086006]; is part of membrane depolarization during bundle of His cell action potential [GO:0086048] Sources: GOC:BHF, GOC:mtg_cardiac_conduct_nov11